{
  "term_id": "GO:0005198",
  "gene_name": "LYR motif-containing protein 4",
  "term_label": "structural molecule activity",
  "gene": "UniProtKB:Q9HD34",
  "gene_symbol": "LYRM4"
}